{
  "gene": "UniProtKB:Q7Z3D4",
  "gene_name": "LysM and putative peptidoglycan-binding domain-containing protein 3",
  "term_id": "GO:0005794",
  "term_label": "Golgi apparatus",
  "gene_symbol": "LYSMD3"
}